{
  "gene": "UniProtKB:Q96CW9",
  "gene_name": "Netrin-G2",
  "term_label": "synaptic membrane adhesion",
  "term_id": "GO:0099560",
  "gene_symbol": "NTNG2"
}